{
  "gene": "UniProtKB:Q86VP6",
  "term_id": "UNKNOWN:0001",
  "gene_symbol": "CAND1",
  "gene_name": "Cullin-associated NEDD8-dissociated protein 1",
  "term_label": "Unknown molecular function"
}